negative regulation of mRNA cis splicing, via spliceosome [GO:1905745] (biological process) Definition: Any process that stops, prevents or reduces the frequency, rate or extent of mRNA cis splicing, via spliceosome. References: PMID:2880558 Sources: GOC:TermGenie, GO_REF:0000058 Relationships: is a type of negative regulation of mRNA splicing, via spliceosome [GO:0048025]; is a type of regulation of mRNA cis splicing, via spliceosome [GO:1905744]; negatively regulates mRNA cis splicing, via spliceosome [GO:0045292]